{
  "gene_symbol": "MAML2",
  "gene": "UniProtKB:Q8IZL2",
  "term_id": "GO:0005654",
  "term_label": "nucleoplasm",
  "gene_name": "Mastermind-like protein 2"
}